{
  "gene_name": "Uncharacterized protein encoded by LINC01548",
  "term_label": "Unknown cellular component",
  "term_id": "UNKNOWN:0003",
  "gene": "UniProtKB:A6NM66",
  "gene_symbol": "LINC01548"
}